{
  "term_label": "RNA polymerase II cis-regulatory region sequence-specific DNA binding",
  "term_id": "GO:0000978",
  "gene": "UniProtKB:Q6PK81",
  "gene_name": "Zinc finger protein 773",
  "gene_symbol": "ZNF773"
}